{
  "gene_name": "Liprin-beta-2",
  "gene_symbol": "PPFIBP2",
  "term_id": "GO:0007528",
  "gene": "UniProtKB:Q8ND30",
  "term_label": "neuromuscular junction development"
}